nuclear retinoid X receptor binding [GO:0046965] (MF) Relationships: is a type of nuclear retinoic acid receptor binding [GO:0042974] Definition: Binding to a nuclear retinoid X receptor. Also known as: retinoid X receptor binding, RXR binding Sources: GOC:ai